3-(imidazol-5-yl)lactate dehydrogenase activity [GO:0019155] (molecular function) Sources: EC:1.1.1.111 Relationships: is a type of GO:0016616 Also known as: (S)-3-(imidazol-5-yl)lactate:NAD(P)+ oxidoreductase activity, imidazol-5-yl lactate dehydrogenase activity Definition: Catalysis of the reaction: (S)-3-(imidazol-5-yl)lactate + NADP+ = 3-(imidazol-5-yl)pyruvate + NADPH + H+.